L-glutamate catabolic process to propionate [GO:0033509] (biological process) Also known as: glutamate breakdown to propionate, glutamate degradation to propionate Sources: GOC:mah, MetaCyc:PWY-5088 Relationships: is a type of L-glutamate catabolic process [GO:0006538]; is a type of propionate metabolic process [GO:0019541] Definition: The chemical reactions and pathways resulting in the breakdown of L-glutamate into other compounds, including propionate.